{
  "term_id": "GO:0004482",
  "gene_name": "mRNA cap guanine-N7 methyltransferase",
  "gene": "UniProtKB:O43148",
  "gene_symbol": "RNMT",
  "term_label": "mRNA 5'-cap (guanine-N7-)-methyltransferase activity"
}